{
  "gene": "UniProtKB:Q9NQV8",
  "gene_symbol": "PRDM8",
  "term_label": "nucleus",
  "gene_name": "PR domain zinc finger protein 8",
  "term_id": "GO:0005634"
}